{
  "gene_symbol": "SYVN1",
  "gene_name": "E3 ubiquitin-protein ligase synoviolin",
  "gene": "UniProtKB:Q86TM6",
  "term_label": "endoplasmic reticulum quality control compartment",
  "term_id": "GO:0044322"
}